hepatocyte growth factor production [GO:0032605] (biological process) Relationships: is a type of cytokine production [GO:0001816]; is a type of protein metabolic process [GO:0019538] References: PMID:1838014 Sources: GOC:mah Also known as: HGF production, scatter factor production, hepatocyte growth factor biosynthetic process Regulation: regulated by regulation of hepatocyte growth factor production [GO:0032646]; negatively regulated by negative regulation of hepatocyte growth factor production [GO:0032686]; positively regulated by positive regulation of hepatocyte growth factor production [GO:0032726] Definition: The appearance of hepatocyte growth factor due to biosynthesis or secretion following a cellular stimulus, resulting in an increase in its intracellular or extracellular levels.